mesenchymal stem cell differentiation involved in metanephric nephron morphogenesis [GO:0072281] (biological process) Definition: The process in which a relatively unspecialized cell acquires specialized features of a mesenchymal stem cell that contributes to the shaping of a nephronin the metanephros. A mesenchymal stem cell is a cell that retains the ability to divide and proliferate throughout life to provide progenitor cells that can differentiate into specialized mesenchymal cells. Sources: GOC:mtg_kidney_jan10 Relationships: is a type of cell differentiation involved in mesonephros development [GO:0061208]; is a type of GO:0072037; is a type of cell differentiation involved in metanephros development [GO:0072202]; is part of metanephric nephron morphogenesis [GO:0072273]